{
  "term_id": "GO:0035861",
  "term_label": "site of double-strand break",
  "gene_symbol": "SETMAR",
  "gene": "UniProtKB:Q53H47",
  "gene_name": "Histone-lysine N-methyltransferase SETMAR"
}